{
  "term_label": "L-valine catabolic process",
  "term_id": "GO:0006574",
  "gene": "UniProtKB:P31937",
  "gene_name": "3-hydroxyisobutyrate dehydrogenase, mitochondrial",
  "gene_symbol": "HIBADH"
}